{
  "gene_symbol": "EP300",
  "gene": "UniProtKB:Q09472",
  "term_label": "transcription regulator complex",
  "term_id": "GO:0005667",
  "gene_name": "Histone acetyltransferase p300"
}